{
  "term_label": "Unknown biological process",
  "gene_name": "Olfactory receptor 52E6",
  "gene": "UniProtKB:Q96RD3",
  "term_id": "UNKNOWN:0002",
  "gene_symbol": "OR52E6"
}